{
  "term_label": "potassium ion transmembrane transport",
  "term_id": "GO:0071805",
  "gene": "UniProtKB:O60706",
  "gene_name": "ATP-binding cassette sub-family C member 9",
  "gene_symbol": "ABCC9"
}